{
  "term_label": "transmembrane signaling receptor activity",
  "gene_symbol": "A0A1W2PQF6",
  "gene_name": "Immunoglobulin subtype domain-containing protein",
  "gene": "UniProtKB:A0A1W2PQF6",
  "term_id": "GO:0004888"
}